{
  "term_id": "UNKNOWN:0002",
  "gene_symbol": "OR51B4",
  "term_label": "Unknown biological process",
  "gene": "UniProtKB:Q9Y5P0",
  "gene_name": "Olfactory receptor 51B4"
}